{
  "gene_symbol": "MEIKIN",
  "gene_name": "Meiosis-specific kinetochore protein",
  "term_label": "Unknown cellular component",
  "term_id": "UNKNOWN:0003",
  "gene": "UniProtKB:A0A087WXM9"
}